{
  "gene_name": "Pulmonary surfactant-associated protein C",
  "term_id": "GO:0005615",
  "gene_symbol": "SFTPC",
  "gene": "UniProtKB:P11686",
  "term_label": "extracellular space"
}